{
  "term_label": "plasma membrane",
  "term_id": "GO:0005886",
  "gene_symbol": "SCN4B",
  "gene": "UniProtKB:Q8IWT1",
  "gene_name": "Sodium channel subunit beta-4"
}